condensed chromatin of inactivated sex chromosome [GO:0098578] (cellular component) Sources: GOC:dos Definition: A condensed form of chromatin that is associated with an inactivated sex chromosome and which is responsible for its inactivation. Relationships: is a type of GO:0001739; is part of inactive sex chromosome [GO:0098577]